{
  "gene_symbol": "XNDC1N",
  "gene_name": "Protein XNDC1N",
  "gene": "UniProtKB:Q6ZNB5",
  "term_label": "Unknown cellular component",
  "term_id": "UNKNOWN:0003"
}